GC-box binding [GO:0140728] (molecular function) Definition: Binding to a GC-box, a DNA motif with the consensus sequence GGGCGG that is located upstream of the start point of eukaryotic transcription units. The GC-box may occur in multiple copies or in either orientation relative to the transcription start site. Relationships: is a type of GO:0000978 References: PMID:14701757 Also known as: GC rich promoter region binding, GC-rich region binding, GC_rich_promoter_region binding, GC box binding